gastric motility [GO:0035482] (biological process) Definition: The spontaneous peristaltic movements of the stomach that aid in digestion, moving food through the stomach and out through the pyloric sphincter into the duodenum. Subtypes: GO:0035483 Regulation: regulated by GO:1905333 References: PMID:16139031 Sources: GOC:cy, ISBN:9781416032458 Relationships: is a type of digestive system process [GO:0022600]